{
  "gene_name": "Complement C1q-like protein 2",
  "term_id": "GO:0099550",
  "gene": "UniProtKB:Q7Z5L3",
  "term_label": "trans-synaptic signaling, modulating synaptic transmission",
  "gene_symbol": "C1QL2"
}